{
  "term_label": "Unknown cellular component",
  "term_id": "UNKNOWN:0003",
  "gene_symbol": "DLG5",
  "gene_name": "Disks large homolog 5",
  "gene": "UniProtKB:Q8TDM6"
}